positive regulation of synaptic transmission, cholinergic [GO:0032224] (biological process) Definition: Any process that activates, maintains or increases the frequency, rate or extent of cholinergic synaptic transmission, the process of communication from a neuron to another neuron across a synapse using the neurotransmitter acetylcholine. Sources: GOC:mah Also known as: up regulation of synaptic transmission, cholinergic, up-regulation of synaptic transmission, cholinergic, upregulation of synaptic transmission, cholinergic, activation of synaptic transmission, cholinergic, stimulation of synaptic transmission, cholinergic Relationships: is_a GO:0032222; is a type of GO:0050806; RO_0002213 GO:0007271 Subtypes: positive regulation of acetylcholine secretion, neurotransmission [GO:0014057]